defense response [GO:0006952] (biological process) Sources: GOC:go_curators Relationships: is a type of response to stress [GO:0006950] Also known as: defence response, physiological defense response, antimicrobial peptide activity, defense/immunity protein activity Subtypes: behavioral defense response [GO:0002209], defense response to insect [GO:0002213], GO:0002215, GO:0002229, GO:0002357, inflammatory response [GO:0006954], cellular defense response [GO:0006968], defense response to bacterium [GO:0042742], defense response to fungus [GO:0050832], defense response to virus [GO:0051607], GO:0052482, GO:0052542, defense response to other organism [GO:0098542] Definition: Reactions, triggered in response to the presence of a foreign body or the occurrence of an injury, which result in restriction of damage to the organism attacked or prevention/recovery from the infection caused by the attack. Regulation: regulated by regulation of defense response [GO:0031347]; negatively regulated by negative regulation of defense response [GO:0031348]; positively regulated by positive regulation of defense response [GO:0031349]